{
  "term_id": "GO:0042273",
  "term_label": "ribosomal large subunit biogenesis",
  "gene_name": "Probable rRNA-processing protein EBP2",
  "gene_symbol": "EBNA1BP2",
  "gene": "UniProtKB:Q99848"
}